{
  "gene_symbol": "PRDM11",
  "term_id": "GO:0005737",
  "gene": "UniProtKB:Q9NQV5",
  "term_label": "cytoplasm",
  "gene_name": "PR domain-containing protein 11"
}